{
  "term_label": "thiamine pyrophosphate transmembrane transport",
  "gene_name": "Mitochondrial thiamine pyrophosphate carrier",
  "gene": "UniProtKB:Q9HC21",
  "gene_symbol": "SLC25A19",
  "term_id": "GO:0030974"
}